{
  "gene_symbol": "TOP2A",
  "gene_name": "DNA topoisomerase 2-alpha",
  "term_id": "GO:0030263",
  "gene": "UniProtKB:P11388",
  "term_label": "apoptotic chromosome condensation"
}